stereocilia ankle link [GO:0002141] (cellular component) Relationships: is a type of GO:0002139 References: PMID:17567809 Definition: A stereocilia coupling link that is composed of a fine filament present in developing stereocilia that couples the bases of individual stereocilia to one another. They are not present in mature stereocilia.